{
  "gene_name": "Nucleoplasmin-2",
  "term_label": "cytoplasm",
  "gene_symbol": "NPM2",
  "gene": "UniProtKB:Q86SE8",
  "term_id": "GO:0005737"
}